{
  "gene_symbol": "TRPC6",
  "term_label": "regulation of cytosolic calcium ion concentration",
  "gene": "UniProtKB:Q9Y210",
  "term_id": "GO:0051480",
  "gene_name": "Short transient receptor potential channel 6"
}